homoserine catabolic process [GO:0009091] (biological process) Definition: The chemical reactions and pathways resulting in the breakdown of homoserine, alpha-amino-gamma-hydroxybutyric acid. Sources: GOC:go_curators, ISBN:0198506732 Also known as: homoserine breakdown, homoserine catabolism, homoserine degradation Relationships: is a type of homoserine metabolic process [GO:0009092]; is a type of carboxylic acid catabolic process [GO:0046395]